{
  "term_id": "GO:0006897",
  "gene": "UniProtKB:Q9ULV0",
  "term_label": "endocytosis",
  "gene_symbol": "MYO5B",
  "gene_name": "Unconventional myosin-Vb"
}